{
  "term_id": "GO:0000978",
  "gene_symbol": "TGIF2LX",
  "gene_name": "Homeobox protein TGIF2LX",
  "gene": "UniProtKB:Q8IUE1",
  "term_label": "RNA polymerase II cis-regulatory region sequence-specific DNA binding"
}